positive regulation of germ cell proliferation [GO:1905938] (biological process) Definition: Any process that activates or increases the frequency, rate or extent of germ cell proliferation. Subtypes: GO:2000256 References: PMID:15342467 Sources: GOC:TermGenie, GO_REF:0000058 Also known as: up regulation of germ cell proliferation, up-regulation of germ cell proliferation, upregulation of germ cell proliferation, activation of germ cell proliferation Relationships: is a type of positive regulation of cell population proliferation [GO:0008284]; is a type of positive regulation of multicellular organismal process [GO:0051240]; is_a GO:1905936; positively regulates germ cell proliferation [GO:0036093]